{
  "term_label": "U4 snRNA 3'-end processing",
  "term_id": "GO:0034475",
  "gene_symbol": "EXOSC6",
  "gene_name": "Exosome complex component MTR3",
  "gene": "UniProtKB:Q5RKV6"
}